{
  "term_id": "GO:0009306",
  "gene_symbol": "CTAGE4",
  "term_label": "protein secretion",
  "gene_name": "cTAGE family member 4",
  "gene": "UniProtKB:Q8IX94"
}